11-beta-hydroxysteroid dehydrogenase (NAD+) activity [GO:0070523] (molecular function) Relationships: is a type of steroid dehydrogenase activity, acting on the CH-OH group of donors, NAD or NADP as acceptor [GO:0033764] Definition: Catalysis of the reaction: an 11-beta-hydroxysteroid + NAD+ = an 11-oxosteroid + NADH + H+. References: PMID:15761036 Sources: RHEA:53116